{
  "term_id": "GO:0071786",
  "gene_symbol": "REEP3",
  "gene_name": "Receptor expression-enhancing protein 3",
  "gene": "UniProtKB:Q6NUK4",
  "term_label": "endoplasmic reticulum tubular network organization"
}